{
  "term_id": "GO:0005615",
  "gene_name": "Lipocalin-1",
  "term_label": "extracellular space",
  "gene_symbol": "LCN1",
  "gene": "UniProtKB:P31025"
}